{
  "term_label": "microtubule",
  "gene": "UniProtKB:Q2TAC6",
  "gene_name": "Kinesin-like protein KIF19",
  "term_id": "GO:0005874",
  "gene_symbol": "KIF19"
}